{
  "gene": "UniProtKB:Q5VWJ9",
  "term_id": "GO:0000407",
  "gene_name": "Sorting nexin-30",
  "term_label": "phagophore assembly site",
  "gene_symbol": "SNX30"
}